{
  "gene": "UniProtKB:A6NHA9",
  "term_label": "olfactory receptor activity",
  "gene_name": "Olfactory receptor 4C46",
  "term_id": "GO:0004984",
  "gene_symbol": "OR4C46"
}